{
  "gene_name": "Polypeptide N-acetylgalactosaminyltransferase 5",
  "term_label": "protein O-linked glycosylation",
  "term_id": "GO:0006493",
  "gene": "UniProtKB:Q7Z7M9",
  "gene_symbol": "GALNT5"
}